{
  "term_label": "ATP binding",
  "gene_symbol": "P2RY1",
  "gene_name": "P2Y purinoceptor 1",
  "term_id": "GO:0005524",
  "gene": "UniProtKB:P47900"
}